{
  "gene_name": "Beta-defensin 107",
  "gene": "UniProtKB:Q8IZN7",
  "gene_symbol": "DEFB107A",
  "term_label": "Unknown cellular component",
  "term_id": "UNKNOWN:0003"
}